maintenance of floral organ identity [GO:0048497] (biological process) Definition: The process in which the identity of a floral organ is maintained. Identity is considered to be the aggregate of characteristics by which a structure is recognized. Relationships: is a type of maintenance of plant organ identity [GO:0090700]; is part of floral organ development [GO:0048437] References: PMID:9090883 Sources: GOC:PO_curators, GOC:tair_curators, PO:0025395